{
  "term_id": "GO:0005102",
  "term_label": "signaling receptor binding",
  "gene_name": "Na(+)_H(+) exchange regulatory cofactor NHE-RF4",
  "gene": "UniProtKB:Q86UT5",
  "gene_symbol": "NHERF4"
}